{
  "gene_symbol": "ARID4B",
  "gene": "UniProtKB:Q4LE39",
  "term_label": "nucleus",
  "term_id": "GO:0005634",
  "gene_name": "AT-rich interactive domain-containing protein 4B"
}